{
  "gene_name": "Polyribonucleotide nucleotidyltransferase 1, mitochondrial",
  "term_label": "cytosol",
  "gene": "UniProtKB:Q8TCS8",
  "gene_symbol": "PNPT1",
  "term_id": "GO:0005829"
}